{
  "gene": "UniProtKB:Q5VSR9",
  "term_label": "Unknown biological process",
  "gene_symbol": "SPANXN1",
  "gene_name": "Sperm protein associated with the nucleus on the X chromosome N1",
  "term_id": "UNKNOWN:0002"
}